{
  "gene_name": "S-adenosylmethionine sensor upstream of mTORC1",
  "term_label": "Unknown molecular function",
  "gene": "UniProtKB:Q1RMZ1",
  "term_id": "UNKNOWN:0001",
  "gene_symbol": "BMT2"
}